kynureninase activity [GO:0030429] (molecular function) References: PMID:17300176 Sources: EC:3.7.1.3 Relationships: is a type of GO:0016823 Also known as: L-kynurenine hydrolase activity, kynurenine hydrolase activity Definition: Catalysis of the reaction: L-kynurenine + H2O = anthranilate + L-alanine + H+. Also acts on 3'-hydroxykynurenine and some other (3-arylcarbonyl)- alanines.